{
  "term_id": "UNKNOWN:0003",
  "gene_name": "Immunoglobulin lambda joining 1",
  "gene": "UniProtKB:A0A0A0MT76",
  "term_label": "Unknown cellular component",
  "gene_symbol": "IGLJ1"
}